{
  "term_id": "GO:0005615",
  "term_label": "extracellular space",
  "gene_symbol": "IL15",
  "gene": "UniProtKB:P40933",
  "gene_name": "Interleukin-15"
}